1-aminocyclopropane-1-carboxylate deaminase activity [GO:0008660] (molecular function) Sources: RHEA:16933 Relationships: is a type of GO:0019239 Also known as: 1-aminocyclopropane carboxylic acid deaminase activity, 1-aminocyclopropane-1-carboxylate aminohydrolase (isomerizing), 1-aminocyclopropane-1-carboxylate endolyase (deaminating) activity, ACC deaminase activity Definition: Catalysis of the reaction: 1-aminocyclopropane-1-carboxylate + H2O = 2-oxobutanate + NH4.